{
  "gene": "UniProtKB:Q5JWF2",
  "term_id": "GO:0031698",
  "gene_symbol": "GNAS",
  "term_label": "beta-2 adrenergic receptor binding",
  "gene_name": "Guanine nucleotide-binding protein G(s) subunit alpha isoforms XLas"
}